{
  "gene_symbol": "IER3IP1",
  "term_id": "GO:0006888",
  "gene": "UniProtKB:Q9Y5U9",
  "term_label": "endoplasmic reticulum to Golgi vesicle-mediated transport",
  "gene_name": "Immediate early response 3-interacting protein 1"
}